{
  "gene_name": "Receptor activity-modifying protein 1",
  "term_id": "GO:0032870",
  "term_label": "cellular response to hormone stimulus",
  "gene": "UniProtKB:O60894",
  "gene_symbol": "RAMP1"
}